{
  "gene": "UniProtKB:O75487",
  "term_id": "GO:0098696",
  "gene_symbol": "GPC4",
  "term_label": "regulation of neurotransmitter receptor localization to postsynaptic specialization membrane",
  "gene_name": "Glypican-4"
}